retrograde trans-synaptic signaling by endocannabinoid [GO:0098921] (biological process) Definition: Cell-cell signaling from postsynapse to presynapse, across the synaptic cleft, mediated by an endocannabinoid ligand. Sources: GOC:dos Relationships: is a type of GO:0098920; is a type of trans-synaptic signaling by endocannabinoid [GO:0099542] Regulation: regulated by regulation of retrograde trans-synaptic signaling by endocanabinoid [GO:0099178]